{
  "gene_symbol": "SCG5",
  "term_label": "regulation of hormone secretion",
  "gene": "UniProtKB:P05408",
  "term_id": "GO:0046883",
  "gene_name": "Neuroendocrine protein 7B2"
}